meiotic DNA double-strand break processing [GO:0000706] (biological process) References: PMID:9334324 Sources: GOC:elh Subtypes: meiotic DNA double-strand break processing involved in meiotic gene conversion [GO:0010704], GO:0010705 Relationships: is a type of DNA double-strand break processing [GO:0000729]; is a type of meiotic cell cycle process [GO:1903046] Definition: The cell cycle process in which the 5' to 3' exonucleolytic resection of the DNA at the site of the break to form a 3' single-strand DNA overhang occurs. This takes place during meiosis.